{
  "gene": "UniProtKB:Q96PG8",
  "term_label": "mitochondrion",
  "gene_name": "Bcl-2-binding component 3, isoforms 3_4",
  "term_id": "GO:0005739",
  "gene_symbol": "BBC3"
}